{
  "gene_symbol": "TNFRSF9",
  "gene_name": "Tumor necrosis factor receptor superfamily member 9",
  "term_label": "regulation of cell population proliferation",
  "gene": "UniProtKB:Q07011",
  "term_id": "GO:0042127"
}